CCR4-NOT complex binding [GO:1905762] (molecular function) Definition: Binding to a CCR4-NOT complex. Relationships: is a type of protein-containing complex binding [GO:0044877] References: PMID:26942678 Sources: GOC:TermGenie